{
  "gene_name": "Protein yippee-like 1",
  "term_label": "Unknown biological process",
  "term_id": "UNKNOWN:0002",
  "gene_symbol": "YPEL1",
  "gene": "UniProtKB:O60688"
}